{
  "term_id": "UNKNOWN:0003",
  "gene_name": "Immunoglobulin heavy variable 4-61",
  "gene": "UniProtKB:A0A0C4DH41",
  "term_label": "Unknown cellular component",
  "gene_symbol": "IGHV4-61"
}